{
  "gene_name": "Histone acetyltransferase KAT6A",
  "term_label": "regulation of transcription by RNA polymerase II",
  "term_id": "GO:0006357",
  "gene_symbol": "KAT6A",
  "gene": "UniProtKB:Q92794"
}